{
  "term_label": "potassium ion transmembrane transport",
  "term_id": "GO:0071805",
  "gene_symbol": "SLC9A8",
  "gene": "UniProtKB:Q9Y2E8",
  "gene_name": "Sodium_hydrogen exchanger 8"
}